{
  "gene_symbol": "ACYP1",
  "gene": "UniProtKB:P07311",
  "gene_name": "Acylphosphatase-1",
  "term_id": "GO:0003998",
  "term_label": "acylphosphatase activity"
}